inferior olivary nucleus formation [GO:0021715] (biological process) Relationships: is a type of anatomical structure formation involved in morphogenesis [GO:0048646]; is part of medulla oblongata formation [GO:0021580]; is part of inferior olivary nucleus morphogenesis [GO:0021714] Also known as: inferior olive biosynthesis, inferior olive formation Sources: GOC:cls, GOC:dgh, GOC:dph, GOC:jid, GO_REF:0000021 Definition: The process that gives rise to the inferior olivary nucleus. This process pertains to the initial formation of a structure from unspecified parts. The inferior olivary nucleus is a capsule-shaped structure in the ventral medulla located just lateral and dorsal to the medullary pyramids. Neurons in the inferior olivary nucleus are the source of climbing fiber input to the cerebellar cortex; these neurons have been implicated in various functions, such as learning and timing of movements.